{
  "gene": "UniProtKB:Q9HB31",
  "gene_symbol": "SEBOX",
  "term_label": "Unknown molecular function",
  "gene_name": "Homeobox protein SEBOX",
  "term_id": "UNKNOWN:0001"
}